cellular response to leptin stimulus [GO:0044320] (biological process) Definition: Any process that results in a change in state or activity of a cell (in terms of movement, secretion, enzyme production, gene expression, etc.) as a result of a leptin stimulus. Leptin is a hormone manufactured primarily in the adipocytes of white adipose tissue, and the level of circulating leptin is directly proportional to the total amount of fat in the body. It plays a key role in regulating energy intake and energy expenditure, including appetite and metabolism. Sources: GOC:yaf Relationships: is a type of cellular response to hormone stimulus [GO:0032870]; is a type of response to leptin [GO:0044321]